endothelial cell morphogenesis [GO:0001886] (BP) Relationships: is a type of epithelial cell morphogenesis [GO:0003382]; is part of endothelial cell development [GO:0001885] Definition: The change in form (cell shape and size) that occurs during the differentiation of an endothelial cell. Sources: GOC:ascb_2009, GOC:dph, GOC:tb